{
  "gene_name": "Armadillo repeat-containing X-linked protein 3",
  "term_id": "GO:0019896",
  "gene": "UniProtKB:Q9UH62",
  "term_label": "axonal transport of mitochondrion",
  "gene_symbol": "ARMCX3"
}